{
  "gene_symbol": "HSP90B2P",
  "term_id": "GO:0005743",
  "gene": "UniProtKB:Q58FF3",
  "term_label": "mitochondrial inner membrane",
  "gene_name": "Putative endoplasmin-like protein"
}